{
  "term_label": "regulation of transcription by RNA polymerase II",
  "gene_name": "Transcriptional activator protein Pur-alpha",
  "gene": "UniProtKB:Q00577",
  "gene_symbol": "PURA",
  "term_id": "GO:0006357"
}